{
  "gene_symbol": "SCD",
  "term_id": "GO:0005506",
  "gene_name": "Stearoyl-CoA desaturase",
  "gene": "UniProtKB:O00767",
  "term_label": "iron ion binding"
}